thioethanolamine S-acetyltransferase activity [GO:0050336] (molecular function) Relationships: is a type of S-acetyltransferase activity [GO:0016418] Definition: Catalysis of the reaction: acetyl-CoA + cysteamine = S-acetylcysteamine + CoA. Sources: EC:2.3.1.11, RHEA:23280 Also known as: acetyl-CoA:2-aminoethanethiol S-acetyltransferase activity, acetyl-CoA:thioethanolamine S-acetyltransferase activity, thioethanolamine acetyltransferase activity, thioltransacetylase B activity